{
  "term_label": "Unknown cellular component",
  "gene_symbol": "PIERCE1",
  "gene_name": "Piercer of microtubule wall 1 protein",
  "term_id": "UNKNOWN:0003",
  "gene": "UniProtKB:Q5BN46"
}